CDP-choline pathway [GO:0006657] (biological process) Relationships: is a type of phosphatidylcholine biosynthetic process [GO:0006656]; has part choline kinase activity [GO:0004103]; has part diacylglycerol cholinephosphotransferase activity [GO:0004142] Also known as: Kennedy pathway, phosphatidylcholine biosynthesis from choline Sources: ISBN:0471331309, MetaCyc:PWY3O-450 Definition: The phosphatidylcholine biosynthetic process that begins with the phosphorylation of choline and ends with the combination of CDP-choline with diacylglycerol to form phosphatidylcholine.